camalexin biosynthetic process [GO:0010120] (biological process) Definition: The chemical reactions and pathways resulting in the formation of camalexin, an indole phytoalexin. Sources: GOC:pz Also known as: camalexin anabolism, camalexin biosynthesis, camalexin formation, camalexin synthesis Relationships: is a type of indole phytoalexin biosynthetic process [GO:0009700]; is a type of sulfur compound biosynthetic process [GO:0044272] Regulation: positively regulated by positive regulation of camalexin biosynthetic process [GO:1901183]